cyclohex-1-ene-1-carboxyl-CoA hydratase activity [GO:0018811] (molecular function) Relationships: is a type of hydro-lyase activity [GO:0016836] Definition: Catalysis of the reaction: cyclohex-1-ene-1-carboxyl-CoA + H2O = 2-hydroxycyclohexane-1-carboxyl-CoA. Sources: MetaCyc:R266-RXN, UM-BBD_reactionID:r0191